{
  "gene_symbol": "PRELID2",
  "term_label": "mitochondrial intermembrane space",
  "gene": "UniProtKB:Q8N945",
  "gene_name": "PRELI domain-containing protein 2",
  "term_id": "GO:0005758"
}